regulation of protein localization to kinetochore [GO:1905340] (biological process) Subtypes: negative regulation of protein localization to kinetochore [GO:1905341], positive regulation of protein localization to kinetochore [GO:1905342] References: PMID:22581055 Sources: GOC:TermGenie, GO_REF:0000058 Relationships: is a type of regulation of protein localization [GO:0032880]; regulates protein localization to kinetochore [GO:0034501] Definition: Any process that modulates the frequency, rate or extent of protein localization to kinetochore. Also known as: regulation of protein localisation to kinetochore, regulation of condensin localization to kinetochore Note: Q9H211 in Human in PMID:22581055